{
  "gene_name": "Meiosis-specific with OB domain-containing protein",
  "term_id": "GO:0003697",
  "gene_symbol": "MEIOB",
  "term_label": "single-stranded DNA binding",
  "gene": "UniProtKB:Q8N635"
}